{
  "gene_name": "Coiled-coil domain-containing protein 122",
  "term_label": "Unknown cellular component",
  "gene_symbol": "CCDC122",
  "gene": "UniProtKB:Q5T0U0",
  "term_id": "UNKNOWN:0003"
}